regulation of mitotic cell cycle DNA replication [GO:1903463] (biological process) Definition: Any process that modulates the frequency, rate or extent of mitotic cell cycle DNA replication. References: PMID:1234 Sources: GOC:TermGenie, GOC:mtg_cell_cycle, GO_REF:0000058 Subtypes: negative regulation of mitotic cell cycle DNA replication [GO:1903464], positive regulation of mitotic cell cycle DNA replication [GO:1903465], GO:1903466 Also known as: regulation of DNA replication involved in S phase involved in mitotic cell cycle, regulation of DNA replication involved in S-phase involved in mitotic cell cycle, regulation of mitotic nuclear cell cycle DNA replication, regulation of DNA replication during S phase involved in mitotic cell cycle, regulation of nuclear cell cycle DNA replication involved in mitotic cell cycle Relationships: is a type of GO:0007346; is a type of regulation of nuclear cell cycle DNA replication [GO:0033262]; regulates mitotic DNA replication [GO:1902969]